{
  "term_id": "UNKNOWN:0003",
  "gene_name": "tRNA (guanine(6)-N2)-methyltransferase THUMP3",
  "term_label": "Unknown cellular component",
  "gene_symbol": "THUMPD3",
  "gene": "UniProtKB:Q9BV44"
}